{
  "gene_name": "Tumor necrosis factor receptor superfamily member 6",
  "term_id": "GO:0005031",
  "gene": "UniProtKB:P25445",
  "term_label": "tumor necrosis factor receptor activity",
  "gene_symbol": "FAS"
}